{
  "gene_name": "Cilia- and flagella-associated protein HOATZ",
  "gene_symbol": "HOATZ",
  "gene": "UniProtKB:Q6PI97",
  "term_label": "Unknown biological process",
  "term_id": "UNKNOWN:0002"
}